{
  "gene_symbol": "AKIRIN1",
  "gene": "UniProtKB:Q9H9L7",
  "term_id": "GO:0045663",
  "term_label": "positive regulation of myoblast differentiation",
  "gene_name": "Akirin-1"
}